{
  "gene": "UniProtKB:Q13258",
  "gene_symbol": "PTGDR",
  "gene_name": "Prostaglandin D2 receptor",
  "term_id": "GO:0007204",
  "term_label": "positive regulation of cytosolic calcium ion concentration"
}